{
  "gene": "UniProtKB:Q8NH08",
  "term_id": "GO:0005886",
  "term_label": "plasma membrane",
  "gene_name": "Olfactory receptor 10AC1",
  "gene_symbol": "OR10AC1"
}